{
  "term_id": "GO:0034197",
  "gene": "UniProtKB:P11597",
  "term_label": "triglyceride transport",
  "gene_name": "Cholesteryl ester transfer protein",
  "gene_symbol": "CETP"
}